cellulose binding [GO:0030248] (molecular function) Definition: Binding to cellulose. Sources: GOC:mah Relationships: is a type of polysaccharide binding [GO:0030247]